{
  "term_label": "antigen binding",
  "gene": "UniProtKB:P0DP08",
  "gene_symbol": "IGHV4-38-2",
  "term_id": "GO:0003823",
  "gene_name": "Immunoglobulin heavy variable 4-38-2"
}